{
  "gene": "UniProtKB:Q08AE8",
  "term_label": "cleavage furrow formation",
  "gene_name": "Protein spire homolog 1",
  "term_id": "GO:0036089",
  "gene_symbol": "SPIRE1"
}